{
  "gene_name": "Olfactory receptor 6J1",
  "term_id": "GO:0004984",
  "gene_symbol": "OR6J1",
  "gene": "UniProtKB:Q8NGC5",
  "term_label": "olfactory receptor activity"
}